{
  "term_label": "transcription corepressor activity",
  "gene_symbol": "TBL1XR1",
  "gene": "UniProtKB:Q9BZK7",
  "gene_name": "F-box-like_WD repeat-containing protein TBL1XR1",
  "term_id": "GO:0003714"
}